{
  "gene_symbol": "HADHB",
  "gene": "UniProtKB:P55084",
  "gene_name": "Trifunctional enzyme subunit beta, mitochondrial",
  "term_label": "mitochondrial fatty acid beta-oxidation multienzyme complex",
  "term_id": "GO:0016507"
}